{
  "term_label": "cilium assembly",
  "gene_symbol": "FBF1",
  "term_id": "GO:0060271",
  "gene_name": "Fas-binding factor 1",
  "gene": "UniProtKB:Q8TES7"
}